{
  "gene_name": "DNA mismatch repair protein Msh3",
  "term_id": "GO:0006298",
  "term_label": "mismatch repair",
  "gene": "UniProtKB:P20585",
  "gene_symbol": "MSH3"
}